flagellum attachment zone [GO:0120119] (cellular component) Relationships: is a type of GO:0070161 Note: Note that we deem cilium and microtubule-based flagellum to be equivalent; the primary term name reflects frequency of use. References: PMID:10361731, PMID:16414276, PMID:17945531, PMID:20541452, PMID:25972344, PMID:2606941, PMID:26746239, PMID:26776656 Also known as: FAZ Definition: A network of cytoskeletal and membranous connections responsible for the lateral attachment of the cilium to the cell body in some trypanosomatid species.